{
  "gene_name": "Transmembrane channel-like protein 2",
  "term_label": "vestibular reflex",
  "gene": "UniProtKB:Q8TDI7",
  "term_id": "GO:0060005",
  "gene_symbol": "TMC2"
}